{
  "gene": "UniProtKB:Q9Y2K2",
  "term_label": "tau-protein kinase activity",
  "gene_name": "Serine_threonine-protein kinase SIK3",
  "term_id": "GO:0050321",
  "gene_symbol": "SIK3"
}